{
  "gene": "UniProtKB:Q99584",
  "gene_name": "Protein S100-A13",
  "term_label": "RAGE receptor binding",
  "term_id": "GO:0050786",
  "gene_symbol": "S100A13"
}